positive regulation of cornification [GO:1905717] (biological process) Also known as: up regulation of cornification, up-regulation of cornification, upregulation of cornification, activation of cornification References: PMID:26014679 Sources: GOC:TermGenie, GO_REF:0000058 Relationships: is_a positive regulation of programmed cell death [GO:0043068]; is a type of regulation of cornification [GO:1905715]; positively regulates cornification [GO:0070268] Definition: Any process that activates or increases the frequency, rate or extent of cornification.